{
  "term_id": "GO:0000981",
  "term_label": "DNA-binding transcription factor activity, RNA polymerase II-specific",
  "gene_name": "Homeobox protein SIX1",
  "gene_symbol": "SIX1",
  "gene": "UniProtKB:Q15475"
}